{
  "term_id": "GO:0003729",
  "gene": "UniProtKB:P20042",
  "term_label": "mRNA binding",
  "gene_name": "Eukaryotic translation initiation factor 2 subunit 2",
  "gene_symbol": "EIF2S2"
}